{
  "gene_name": "Protein FAM110B",
  "term_id": "UNKNOWN:0002",
  "gene_symbol": "FAM110B",
  "term_label": "Unknown biological process",
  "gene": "UniProtKB:Q8TC76"
}